mesenchymal stem cell proliferation involved in nephron morphogenesis [GO:0072090] (BP) Regulation: regulated by regulation of mesenchymal stem cell proliferation involved in nephron morphogenesis [GO:0072042] Sources: GOC:mtg_kidney_jan10 Relationships: is_a GO:0097168 Definition: The multiplication or reproduction of mesenchymal stem cells, resulting in the expansion of a stem cell population, that contributes to the shaping of a nephron.